{
  "gene_name": "Protein S100-A9",
  "term_label": "antimicrobial humoral immune response mediated by antimicrobial peptide",
  "term_id": "GO:0061844",
  "gene": "UniProtKB:P06702",
  "gene_symbol": "S100A9"
}